{
  "term_id": "GO:0098839",
  "gene": "UniProtKB:P39086",
  "gene_symbol": "GRIK1",
  "gene_name": "Glutamate receptor ionotropic, kainate 1",
  "term_label": "postsynaptic density membrane"
}